5-epi-aristolochene-1,3-dihydroxylase activity [GO:0102170] (molecular function) Relationships: is a type of GO:0016709 Sources: EC:1.14.14.149, GOC:pz Definition: Catalysis of the reaction: (+)-5-epi-aristolochene + 2 NADPH + 2 H+ + 2 O2 = capsidiol + 2 NADP + 2 H2O.